{
  "gene_name": "FGFR1 oncogene partner 2",
  "term_label": "response to wounding",
  "gene": "UniProtKB:Q9NVK5",
  "term_id": "GO:0009611",
  "gene_symbol": "FGFR1OP2"
}